{
  "gene_name": "ATP-dependent DNA helicase Q1",
  "term_id": "GO:0005694",
  "gene_symbol": "RECQL",
  "gene": "UniProtKB:P46063",
  "term_label": "chromosome"
}